fibroblast growth factor receptor activity [GO:0005007] (molecular function) Sources: GOC:mah Note: Note that this term represents an activity and not a gene product, and should only be used when the receptor binds the ligand FGF. For receptors that bind other growth factors, consider annotating to terms under 'transmembrane signaling receptor activity ; GO:0004888. Relationships: is a type of transmembrane receptor protein tyrosine kinase activity [GO:0004714]; BFO_0000050 fibroblast growth factor receptor signaling pathway [GO:0008543]; has part fibroblast growth factor binding [GO:0017134] Definition: Combining with a fibroblast growth factor receptor ligand and transmitting the signal across the plasma membrane to initiate a change in cell activity. Also known as: FGF receptor activity, FGF-activated receptor activity, FGFR, fibroblast growth factor-activated receptor activity